{
  "gene": "UniProtKB:P56199",
  "gene_name": "Integrin alpha-1",
  "term_id": "GO:0034665",
  "term_label": "integrin alpha1-beta1 complex",
  "gene_symbol": "ITGA1"
}